protein-RNA adaptor activity [GO:0140517] (molecular function) Subtypes: C5-methylcytidine-containing RNA reader activity [GO:0062153], internal N(7)-methylguanine-containing RNA reader activity [GO:0160089], protein-RNA sequence-specific adaptor activity [GO:0160134], protein-tRNA adaptor activity [GO:0180014], N6-methyladenosine-containing RNA reader activity [GO:1990247] Definition: The binding activity of a protein that brings together another protein and an RNA, permitting those molecules to function in a coordinated way. References: PMID:24470144 Relationships: is a type of protein-macromolecule adaptor activity [GO:0030674]